{
  "term_id": "GO:0005615",
  "gene_name": "Cystatin-9",
  "term_label": "extracellular space",
  "gene_symbol": "CST9",
  "gene": "UniProtKB:Q5W186"
}